{
  "gene_symbol": "LAMTOR2",
  "term_id": "GO:0071986",
  "gene_name": "Ragulator complex protein LAMTOR2",
  "gene": "UniProtKB:Q9Y2Q5",
  "term_label": "Ragulator complex"
}